{
  "gene_symbol": "MYH7",
  "gene_name": "Myosin-7",
  "term_label": "myosin II complex",
  "gene": "UniProtKB:P12883",
  "term_id": "GO:0016460"
}